{
  "gene": "UniProtKB:P55795",
  "term_label": "ribonucleoprotein complex",
  "gene_name": "Heterogeneous nuclear ribonucleoprotein H2",
  "term_id": "GO:1990904",
  "gene_symbol": "HNRNPH2"
}